{
  "gene_name": "DDB1- and CUL4-associated factor 13",
  "term_id": "GO:0032040",
  "term_label": "small-subunit processome",
  "gene": "UniProtKB:Q9NV06",
  "gene_symbol": "DCAF13"
}